{
  "term_label": "Unknown molecular function",
  "gene_name": "Histone deacetylase 6",
  "gene_symbol": "HDAC6",
  "gene": "UniProtKB:Q9UBN7",
  "term_id": "UNKNOWN:0001"
}